facioacoustic ganglion morphogenesis [GO:1904836] (biological process) Definition: The developmental process by which an acoustico-facial VII-VIII ganglion complex is generated and organized. References: PMID:18356247 Sources: GOC:PARL, GOC:TermGenie, GOC:bf, GOC:mat, GO_REF:0000083 Also known as: acoustico-facial VII-VIII ganglion complex morphogenesis, acousticofacial ganglion morphogenesis, facio-acoustic ganglion complex VII-VIII morphogenesis, facio-acoustic ganglion morphogenesis, facio-acoustic VII-VIII ganglion complex morphogenesis, facio-acoustic ganglion complex morphogenesis Relationships: is a type of GO:0061559; is part of facioacoustic ganglion development [GO:1903375]